{
  "gene_symbol": "GID4",
  "gene_name": "Glucose-induced degradation protein 4 homolog",
  "term_id": "UNKNOWN:0003",
  "term_label": "Unknown cellular component",
  "gene": "UniProtKB:Q8IVV7"
}